C-X-C motif chemokine 12 receptor activity [GO:0038147] (MF) Definition: Combining with the C-X-C motif chemokine 12 (CXCL12) and transmitting the signal from one side of the membrane to the other to initiate a change in cell activity. Relationships: is a type of C-X-C chemokine receptor activity [GO:0016494]; is part of chemokine (C-X-C motif) ligand 12 signaling pathway [GO:0038146] References: PMID:22204316 Sources: GOC:bf Also known as: CXCL12 receptor activity, stromal cell-derived factor-1 receptor activity, CXCR4, CXCR7, SDF-1 receptor activity